Cbf1-Met4-Met28 complex [GO:0089713] (CC) Definition: A heteromeric complex consisting of Cbf1 and basic leucine zipper (bZIP) containing transcriptional activators, Met4 and Met28, that forms over the sequence TCACGTG in the upstream activating sequence (UAS) of genes involved in sulfur amino acid metabolism, resulting in their transcriptional activation. References: PMID:8665859, PMID:9171357 Relationships: is a type of transcription regulator complex [GO:0005667]